{
  "gene_name": "Transmembrane 4 L6 family member 5",
  "term_label": "Unknown molecular function",
  "term_id": "UNKNOWN:0001",
  "gene": "UniProtKB:O14894",
  "gene_symbol": "TM4SF5"
}